guanidinobutyrase activity [GO:0047971] (molecular function) Definition: Catalysis of the reaction: 4-guanidinobutanoate + H2O = 4-aminobutanoate + urea. Sources: EC:3.5.3.7, RHEA:19501 Also known as: 4-guanidinobutanoate amidinohydrolase activity, 4-guanidinobutyrate amidinobutyrase activity, G-base activity, GBH, gamma-guanidinobutyrate amidinohydrolase activity, gamma-guanidobutyrase activity, guanidinobutyrate ureahydrolase activity Relationships: is a type of hydrolase activity, acting on carbon-nitrogen (but not peptide) bonds, in linear amidines [GO:0016813]